{
  "gene_name": "Dual specificity protein phosphatase 6",
  "gene_symbol": "DUSP6",
  "term_label": "protein tyrosine/threonine phosphatase activity",
  "gene": "UniProtKB:Q16828",
  "term_id": "GO:0008330"
}